{
  "term_id": "UNKNOWN:0003",
  "gene_symbol": "RSU1",
  "gene_name": "Ras suppressor protein 1",
  "term_label": "Unknown cellular component",
  "gene": "UniProtKB:Q15404"
}